{
  "term_label": "nucleus",
  "gene": "UniProtKB:Q9Y603",
  "gene_symbol": "ETV7",
  "term_id": "GO:0005634",
  "gene_name": "Transcription factor ETV7"
}